thyroid gland development [GO:0030878] (biological process) Relationships: is a type of gland development [GO:0048732]; is part of endocrine system development [GO:0035270] Sources: GOC:dgh Definition: The process whose specific outcome is the progression of the thyroid gland over time, from its formation to the mature structure. The thyroid gland is an endoderm-derived gland that produces thyroid hormone.